type II interferon receptor activity [GO:0004906] (molecular function) Definition: Combining with interferon-gamma (a type II interferon) and transmitting the signal from one side of the membrane to the other to initiate a change in cell activity. Also known as: IFN-gamma receptor activity, IFNG receptor activity, interferon-gamma receptor activity Relationships: is a type of GO:0004904; is part of GO:0060333; has part type II interferon binding [GO:0019964] References: PMID:15546383 Sources: GOC:add, GOC:ai, GOC:signaling, ISBN:0126896631